{
  "gene_name": "Cytotoxic and regulatory T-cell molecule",
  "gene": "UniProtKB:O95727",
  "term_id": "GO:0002355",
  "term_label": "detection of tumor cell",
  "gene_symbol": "CRTAM"
}